{
  "gene_symbol": "AUH",
  "gene_name": "Methylglutaconyl-CoA hydratase, mitochondrial",
  "term_label": "mitochondrion",
  "gene": "UniProtKB:Q13825",
  "term_id": "GO:0005739"
}